{
  "term_id": "GO:0001556",
  "term_label": "oocyte maturation",
  "gene": "UniProtKB:Q86SH2",
  "gene_name": "Zygote arrest protein 1",
  "gene_symbol": "ZAR1"
}